{
  "gene_name": "Interleukin-1 alpha",
  "term_id": "GO:0006954",
  "gene": "UniProtKB:P01583",
  "term_label": "inflammatory response",
  "gene_symbol": "IL1A"
}